{
  "term_label": "neuroligin family protein binding",
  "gene_name": "Neurexin-1",
  "term_id": "GO:0097109",
  "gene": "UniProtKB:Q9ULB1",
  "gene_symbol": "NRXN1"
}